{
  "gene_symbol": "RBP1",
  "term_id": "GO:1904768",
  "term_label": "all-trans-retinol binding",
  "gene_name": "Retinol-binding protein 1",
  "gene": "UniProtKB:P09455"
}